embryo development ending in seed dormancy [GO:0009793] (biological process) Subtypes: somatic embryogenesis [GO:0010262], cotyledon development [GO:0048825] Sources: GOC:go_curators, GOC:mtg_sensu Also known as: embryogenesis Definition: The process whose specific outcome is the progression of the embryo over time, from zygote formation to the end of seed dormancy. An example of this process is found in Arabidopsis thaliana. Relationships: is a type of developmental process involved in reproduction [GO:0003006]; is a type of embryo development [GO:0009790]; is part of seed development [GO:0048316]